{
  "term_label": "cytosol",
  "gene_name": "Serine_threonine-protein phosphatase 2A 55 kDa regulatory subunit B delta isoform",
  "gene_symbol": "PPP2R2D",
  "term_id": "GO:0005829",
  "gene": "UniProtKB:Q66LE6"
}